{
  "gene_name": "RNA-binding protein EWS",
  "term_id": "GO:0003723",
  "gene_symbol": "EWSR1",
  "term_label": "RNA binding",
  "gene": "UniProtKB:Q01844"
}